{
  "gene": "UniProtKB:Q9UHP3",
  "gene_name": "Ubiquitin carboxyl-terminal hydrolase 25",
  "gene_symbol": "USP25",
  "term_id": "GO:0004843",
  "term_label": "cysteine-type deubiquitinase activity"
}